{
  "gene": "UniProtKB:P09871",
  "gene_symbol": "C1S",
  "term_label": "serine-type endopeptidase activity",
  "term_id": "GO:0004252",
  "gene_name": "Complement C1s subcomponent"
}